{
  "term_id": "UNKNOWN:0003",
  "gene_name": "Putative ATP-dependent RNA helicase DHX57",
  "gene_symbol": "DHX57",
  "term_label": "Unknown cellular component",
  "gene": "UniProtKB:Q6P158"
}